{
  "term_id": "GO:0140806",
  "gene_symbol": "PARP2",
  "term_label": "NAD+-protein-aspartate ADP-ribosyltransferase activity",
  "gene_name": "Poly [ADP-ribose] polymerase 2",
  "gene": "UniProtKB:Q9UGN5"
}